ossification involved in bone maturation [GO:0043931] (biological process) Sources: GOC:dph, GOC:mah, GOC:mtg_mpo Relationships: is a type of ossification [GO:0001503]; is part of GO:0070977 Also known as: ossification involved in skeletal development, ossification involved in bone modeling Definition: The formation of bone or of a bony substance, or the conversion of fibrous tissue or of cartilage into bone, involved in the progression of the skeleton from its formation to its mature state.